{
  "gene_name": "Bardet-Biedl syndrome 2 protein",
  "gene_symbol": "BBS2",
  "gene": "UniProtKB:Q9BXC9",
  "term_label": "cilium assembly",
  "term_id": "GO:0060271"
}